regulation of proanthocyanidin biosynthetic process [GO:2000029] (BP) Relationships: is a type of GO:1900376; is_a regulation of phenylpropanoid metabolic process [GO:2000762]; regulates proanthocyanidin biosynthetic process [GO:0010023] Definition: Any process that modulates the frequency, rate or extent of proanthocyanidin biosynthetic process. Sources: GOC:obol Also known as: regulation of proanthocyanidin anabolism, regulation of proanthocyanidin biosynthesis, regulation of proanthocyanidin formation, regulation of proanthocyanidin synthesis